INTAC complex [GO:0160232] (cellular component) Also known as: integrator-PP2A complex References: PMID:33243860, PMID:38570683 Relationships: is a type of nuclear protein-containing complex [GO:0140513]; BFO_0000051 integrator complex [GO:0032039] Definition: A protein complex containing Integrator and protein phosphatase 2A core enzyme (PP2A-AC) that stably associates with the C-terminus of RNA polymerase II and promotes premature RNA polymerase II transcription termination.